{
  "gene_name": "Golgi apparatus membrane protein TVP23 homolog B",
  "gene": "UniProtKB:Q9NYZ1",
  "gene_symbol": "TVP23B",
  "term_label": "vesicle-mediated transport",
  "term_id": "GO:0016192"
}